{
  "gene_name": "Coiled-coil domain-containing protein 62",
  "gene": "UniProtKB:Q6P9F0",
  "term_id": "GO:0045944",
  "term_label": "positive regulation of transcription by RNA polymerase II",
  "gene_symbol": "CCDC62"
}